sinapoylglucose-malate O-sinapoyltransferase activity [GO:0016754] (MF) Relationships: is a type of O-sinapoyltransferase activity [GO:0016753] Sources: EC:2.3.1.92, RHEA:12625 Definition: Catalysis of the reaction: (S)-malate + 1-O-sinapoyl-beta-D-glucose = D-glucose + sinapoyl (S)-malate. Also known as: sinapoylglucose:malate sinapoyltransferase activity, 1-O-sinapoyl-beta-D-glucose:(S)-malate O-sinapoyltransferase activity, 1-sinapoylglucose-L-malate sinapoyltransferase activity